{
  "gene_symbol": "CELA2A",
  "gene_name": "Chymotrypsin-like elastase family member 2A",
  "gene": "UniProtKB:P08217",
  "term_id": "GO:0006508",
  "term_label": "proteolysis"
}